{
  "gene": "UniProtKB:P48556",
  "term_id": "GO:0043161",
  "gene_name": "26S proteasome non-ATPase regulatory subunit 8",
  "term_label": "proteasome-mediated ubiquitin-dependent protein catabolic process",
  "gene_symbol": "PSMD8"
}